{
  "gene_name": "DNA replication licensing factor MCM4",
  "gene": "UniProtKB:P33991",
  "gene_symbol": "MCM4",
  "term_id": "GO:0017116",
  "term_label": "single-stranded DNA helicase activity"
}